{
  "term_id": "GO:0007010",
  "gene_symbol": "NAA25",
  "gene_name": "N-alpha-acetyltransferase 25, NatB auxiliary subunit",
  "gene": "UniProtKB:Q14CX7",
  "term_label": "cytoskeleton organization"
}